{
  "gene_name": "Cap-specific mRNA (nucleoside-2'-O-)-methyltransferase 2",
  "gene": "UniProtKB:Q8IYT2",
  "term_id": "GO:0005737",
  "term_label": "cytoplasm",
  "gene_symbol": "CMTR2"
}